negative regulation of calcitonin secretion [GO:1904363] (biological process) Definition: Any process that stops, prevents or reduces the frequency, rate or extent of calcitonin secretion. Also known as: down regulation of calcitonin secretion, down-regulation of calcitonin secretion, downregulation of calcitonin secretion, inhibition of calcitonin secretion References: PMID:11278900 Sources: GOC:TermGenie, GO_REF:0000058 Relationships: is_a negative regulation of peptide hormone secretion [GO:0090278]; is a type of regulation of calcitonin secretion [GO:1904362]; negatively regulates calcitonin secretion [GO:0036161]